citrate secondary active transmembrane transporter activity [GO:0071913] (molecular function) Definition: Enables the transfer of citrate from one side of a membrane to the other, up its concentration gradient. The transporter binds the solute and undergoes a series of conformational changes. Transport works equally well in either direction and is driven by a chemiosmotic source of energy. Secondary active transporters include symporters and antiporters. Sources: GOC:mah, GOC:mtg_transport, GOC:vw Also known as: citrate carrier activity Relationships: is_a tricarboxylate secondary active transmembrane transporter activity [GO:0005371]; is a type of citrate transmembrane transporter activity [GO:0015137] Subtypes: GO:0015515, citrate:proton symporter activity [GO:0015531], citrate:2-oxoglutarate antiporter activity [GO:0180056]